{
  "gene": "UniProtKB:Q7Z2H8",
  "gene_symbol": "SLC36A1",
  "term_label": "proton transmembrane transport",
  "term_id": "GO:1902600",
  "gene_name": "Proton-coupled amino acid transporter 1"
}